{
  "term_id": "UNKNOWN:0002",
  "gene": "UniProtKB:Q9Y267",
  "gene_name": "Solute carrier family 22 member 14",
  "gene_symbol": "SLC22A14",
  "term_label": "Unknown biological process"
}